viral mRNA export from host cell nucleus [GO:0046784] (biological process) Also known as: intronless viral mRNA export from host cell nucleus, intronless viral mRNA export out of nucleus, intronless viral mRNA transport from nucleus to cytoplasm, intronless viral mRNA-nucleus export, intronless viral mRNA export from host nucleus References: PMID:11598019 Definition: The directed movement of intronless viral mRNA from the host nucleus to the cytoplasm for translation. Relationships: is a type of viral process [GO:0016032]; is part of viral gene expression [GO:0019080]